{
  "gene_name": "Mitogen-activated protein kinase kinase kinase 7",
  "gene": "UniProtKB:O43318",
  "term_id": "GO:0006955",
  "term_label": "immune response",
  "gene_symbol": "MAP3K7"
}